{
  "term_label": "Unknown molecular function",
  "term_id": "UNKNOWN:0001",
  "gene": "UniProtKB:P47756",
  "gene_name": "F-actin-capping protein subunit beta",
  "gene_symbol": "CAPZB"
}